{
  "term_label": "neuron migration",
  "gene_symbol": "TRIM46",
  "term_id": "GO:0001764",
  "gene_name": "Tripartite motif-containing protein 46",
  "gene": "UniProtKB:Q7Z4K8"
}